{
  "gene_symbol": "ITGB8",
  "gene_name": "Integrin beta-8",
  "term_label": "integrin-mediated signaling pathway",
  "gene": "UniProtKB:P26012",
  "term_id": "GO:0007229"
}